phenylalanine:proton symporter activity [GO:0015492] (molecular function) Sources: TC:2.A.3.1.1 Definition: Enables the transfer of a solute or solutes from one side of a membrane to the other according to the reaction: phenylalanine(out) + H+(out) = phenylalanine(in) + H+(in). Relationships: is_a amino acid:proton symporter activity [GO:0005280]; is a type of aromatic amino acid:proton symporter activity [GO:0015494] Also known as: phenylalanine:hydrogen symporter activity